{
  "gene_name": "ORC ubiquitin ligase 1",
  "term_label": "chromatin",
  "gene_symbol": "OBI1",
  "term_id": "GO:0000785",
  "gene": "UniProtKB:Q5W0B1"
}